negative regulation of gonad development [GO:1905940] (biological process) References: PMID:15342467 Sources: GOC:TermGenie, GO_REF:0000058 Also known as: down regulation of gonad development, down regulation of gonadogenesis, down-regulation of gonad development, down-regulation of gonadogenesis, downregulation of gonad development, downregulation of gonadogenesis, negative regulation of gonadogenesis, inhibition of gonad development, inhibition of gonadogenesis Subtypes: GO:2000019, GO:2000195 Definition: Any process that stops, prevents or reduces the frequency, rate or extent of gonad development. Relationships: is_a negative regulation of developmental process [GO:0051093]; is a type of negative regulation of multicellular organismal process [GO:0051241]; is a type of regulation of gonad development [GO:1905939]; is a type of negative regulation of reproductive process [GO:2000242]; negatively regulates gonad development [GO:0008406]